positive regulation of gonadotropin secretion [GO:0032278] (biological process) Sources: GOC:mah Definition: Any process that activates or increases the frequency, rate or extent of the regulated release of a gonadotropin. Relationships: is a type of GO:0032276; is a type of positive regulation of hormone secretion [GO:0046887]; is a type of positive regulation of multicellular organismal process [GO:0051240]; positively regulates gonadotropin secretion [GO:0032274] Subtypes: positive regulation of luteinizing hormone secretion [GO:0033686], positive regulation of follicle-stimulating hormone secretion [GO:0046881] Also known as: positive regulation of gonadotrophin secretion, up regulation of gonadotropin secretion, up-regulation of gonadotropin secretion, upregulation of gonadotropin secretion, activation of gonadotropin secretion, stimulation of gonadotropin secretion